{
  "gene_symbol": "FAM9B",
  "gene": "UniProtKB:Q8IZU0",
  "term_label": "Unknown molecular function",
  "term_id": "UNKNOWN:0001",
  "gene_name": "Protein FAM9B"
}